positive regulation of endoplasmic reticulum stress-induced intrinsic apoptotic signaling pathway [GO:1902237] (biological process) Relationships: is a type of regulation of endoplasmic reticulum stress-induced intrinsic apoptotic signaling pathway [GO:1902235]; is a type of GO:1905898; is a type of positive regulation of intrinsic apoptotic signaling pathway [GO:2001244]; positively regulates intrinsic apoptotic signaling pathway in response to endoplasmic reticulum stress [GO:0070059] Also known as: positive regulation of ER stress-induced apoptosis, positive regulation of apoptosis in response to ER stress, positive regulation of apoptosis triggered by ER stress, positive regulation of endoplasmic reticulum stress-induced apoptosis, positive regulation of intrinsic apoptotic signaling pathway in response to endoplasmic reticulum stress, positive regulation of intrinsic apoptotic signaling pathway induced by endoplasmic reticulum stress, up regulation of ER stress-induced apoptosis, up regulation of apoptosis in response to ER stress, up regulation of apoptosis triggered by ER stress, up regulation of endoplasmic reticulum stress-induced apoptosis, up regulation of intrinsic apoptotic signaling pathway in response to endoplasmic reticulum stress, up regulation of intrinsic apoptotic signaling pathway induced by endoplasmic reticulum stress, up-regulation of ER stress-induced apoptosis, up-regulation of apoptosis in response to ER stress, up-regulation of apoptosis triggered by ER stress, up-regulation of endoplasmic reticulum stress-induced apoptosis, up-regulation of intrinsic apoptotic signaling pathway in response to endoplasmic reticulum stress, up-regulation of intrinsic apoptotic signaling pathway induced by endoplasmic reticulum stress, upregulation of ER stress-induced apoptosis, upregulation of apoptosis in response to ER stress, upregulation of apoptosis triggered by ER stress, upregulation of endoplasmic reticulum stress-induced apoptosis, upregulation of intrinsic apoptotic signaling pathway in response to endoplasmic reticulum stress, upregulation of intrinsic apoptotic signaling pathway induced by endoplasmic reticulum stress, activation of ER stress-induced apoptosis, activation of apoptosis in response to ER stress, activation of apoptosis triggered by ER stress, activation of endoplasmic reticulum stress-induced apoptosis, activation of intrinsic apoptotic signaling pathway in response to endoplasmic reticulum stress, activation of intrinsic apoptotic signaling pathway induced by endoplasmic reticulum stress References: PMID:20160352 Sources: GOC:BHF, GOC:TermGenie, GOC:mtg_apoptosis, GOC:rl Definition: Any process that activates or increases the frequency, rate or extent of an endoplasmic reticulum stress-induced intrinsic apoptotic signaling pathway.